oligosaccharide-diphosphodolichol diphosphatase activity [GO:0047430] (molecular function) Sources: EC:3.6.1.44, MetaCyc:3.6.1.44-RXN Definition: Catalysis of the reaction: H2O + oligosaccharide-diphosphodolichol = dolichol-phosphate + oligosaccharide phosphate. Also known as: oligosaccharide-diphosphodolichol pyrophosphatase activity, oligosaccharide-diphosphodolichol phosphodolichohydrolase activity Relationships: is a type of pyrophosphatase activity [GO:0016462]